XMP biosynthetic process [GO:0097293] (biological process) Sources: GOC:yaf Definition: The chemical reactions and pathways resulting in the formation of XMP, xanthosine monophosphate. Relationships: is a type of purine ribonucleotide biosynthetic process [GO:0009152]; is a type of GO:0009168; is a type of XMP metabolic process [GO:0097292] Also known as: XMP anabolism, XMP biosynthesis, XMP formation, XMP synthesis Subtypes: XMP salvage [GO:0032265], 'de novo' XMP biosynthetic process [GO:0097294]